cellular response to sodium phosphate [GO:1904384] (biological process) Relationships: is a type of cellular response to salt [GO:1902075]; is a type of response to sodium phosphate [GO:1904383] References: PMID:24625659 Sources: GOC:TermGenie, GO_REF:0000071 Definition: Any process that results in a change in state or activity of a cell (in terms of movement, secretion, enzyme production, gene expression, etc.) as a result of a sodium phosphate stimulus.